{
  "term_label": "Unknown biological process",
  "gene": "UniProtKB:Q6P7N7",
  "gene_symbol": "TMEM81",
  "term_id": "UNKNOWN:0002",
  "gene_name": "Transmembrane protein 81"
}